{
  "term_id": "GO:0022857",
  "gene": "UniProtKB:Q8TF71",
  "term_label": "transmembrane transporter activity",
  "gene_name": "Monocarboxylate transporter 10",
  "gene_symbol": "SLC16A10"
}